mitochondrial outer membrane permeabilization [GO:0097345] (biological process) Note: BAX and BAK are involved in this process, as reviewed in PMID:21760595 (the human proteins have UniProt symbols Q07812 and Q16611 respectively). References: PMID:21041309 Sources: GOC:BHF, GOC:mtg_apoptosis, GOC:pg Regulation: regulated by regulation of mitochondrial outer membrane permeabilization involved in apoptotic signaling pathway [GO:1901028]; negatively regulated by negative regulation of mitochondrial outer membrane permeabilization involved in apoptotic signaling pathway [GO:1901029]; positively regulated by GO:1901030 Relationships: is_a positive regulation of mitochondrial membrane permeability involved in apoptotic process [GO:1902110]; is part of GO:0097190 Definition: The process by which the mitochondrial outer membrane becomes permeable to the passing of proteins and other molecules from the intermembrane space to the cytosol as part of the apoptotic signaling pathway. Also known as: mitochondrial outer membrane permeabilization during apoptotic cell death, MOMP, mitochondrion outer membrane permeabilization